bilirubin-glucuronoside glucuronosyltransferase activity [GO:0047278] (molecular function) Also known as: bilirubin glucuronoside glucuronosyltransferase activity, bilirubin monoglucuronide transglucuronidase activity, bilirubin-glucuronoside:bilirubin-glucuronoside D-glucuronosyltransferase activity Sources: RHEA:16885 Definition: Catalysis of the reaction: 2 bilirubin-glucuronoside = bilirubin + bilirubin-bisglucuronoside. Relationships: is a type of glucuronosyltransferase activity [GO:0015020]